{
  "gene_symbol": "NUP37",
  "term_id": "UNKNOWN:0001",
  "term_label": "Unknown molecular function",
  "gene": "UniProtKB:Q8NFH4",
  "gene_name": "Nucleoporin Nup37"
}